phagolysosome vesicle lumen [GO:0106174] (cellular component) Relationships: is a type of vacuolar lumen [GO:0005775]; is a type of cytoplasmic vesicle lumen [GO:0060205]; is a type of GO:0097013; is part of phagolysosome [GO:0032010] Definition: The volume enclosed by the membrane of a phagolysosome. References: PMID:29471269 Sources: GOC:pde